{
  "gene": "UniProtKB:A6NJZ7",
  "gene_symbol": "RIMBP3C",
  "term_id": "GO:0009566",
  "gene_name": "RIMS-binding protein 3C",
  "term_label": "fertilization"
}